negative regulation of kinin cascade [GO:0002257] (biological process) Sources: GOC:jal Also known as: down regulation of kinin cascade, down-regulation of kinin cascade, downregulation of kinin cascade, inhibition of kinin cascade Relationships: is a type of regulation of kinin cascade [GO:0002256]; is a type of negative regulation of acute inflammatory response [GO:0002674]; is a type of negative regulation of protein activation cascade [GO:2000258]; RO_0002212 kinin cascade [GO:0002254] Subtypes: negative regulation of tissue kallikrein-kinin cascade [GO:0002546], GO:0002549 Definition: Any process that stops, prevents, or reduces the frequency, rate, or extent of the kinin cascade.